{
  "term_label": "autophagosome membrane",
  "term_id": "GO:0000421",
  "gene_symbol": "GABARAP",
  "gene": "UniProtKB:O95166",
  "gene_name": "Gamma-aminobutyric acid receptor-associated protein"
}